{
  "gene_symbol": "MGAT5",
  "gene_name": "Alpha-1,6-mannosylglycoprotein 6-beta-N-acetylglucosaminyltransferase A",
  "term_label": "Golgi apparatus",
  "term_id": "GO:0005794",
  "gene": "UniProtKB:Q09328"
}